{
  "gene": "UniProtKB:Q9H3M0",
  "gene_name": "Potassium voltage-gated channel subfamily F member 1",
  "gene_symbol": "KCNF1",
  "term_id": "GO:0015459",
  "term_label": "potassium channel regulator activity"
}